CDP-alcohol phosphatidyltransferase activity [GO:0017169] (MF) Subtypes: CDP-diacylglycerol-inositol 3-phosphatidyltransferase activity [GO:0003881], GO:0003882, diacylglycerol cholinephosphotransferase activity [GO:0004142], ethanolaminephosphotransferase activity [GO:0004307], CDP-diacylglycerol-glycerol-3-phosphate 3-phosphatidyltransferase activity [GO:0008444] Relationships: is a type of GO:0016780 Definition: Catalysis of the reaction: CDP + alcohol = CMP + phosphatidyl alcohol. Sources: GOC:ai